{
  "gene_name": "Protein unc-13 homolog B",
  "gene": "UniProtKB:O14795",
  "term_id": "GO:0005516",
  "gene_symbol": "UNC13B",
  "term_label": "calmodulin binding"
}